{
  "gene": "UniProtKB:Q7LGC8",
  "term_label": "Unknown cellular component",
  "gene_symbol": "CHST3",
  "term_id": "UNKNOWN:0003",
  "gene_name": "Carbohydrate sulfotransferase 3"
}